{
  "term_id": "GO:0030424",
  "gene": "UniProtKB:Q9GZV3",
  "term_label": "axon",
  "gene_name": "High affinity choline transporter 1",
  "gene_symbol": "SLC5A7"
}